{
  "term_id": "UNKNOWN:0001",
  "gene": "UniProtKB:H0YL14",
  "term_label": "Unknown molecular function",
  "gene_symbol": "TMEM250",
  "gene_name": "Transmembrane protein 250"
}